hematopoietic stem cell proliferation [GO:0071425] (biological process) Also known as: hemopoietic stem cell proliferation Definition: The expansion of a hematopoietic stem cell population by cell division. A hematopoietic stem cell is a stem cell from which all cells of the lymphoid and myeloid lineages develop. Relationships: is a type of stem cell proliferation [GO:0072089]; is part of hemopoiesis [GO:0030097] Sources: CL:0000037, GOC:BHF, GOC:add, GOC:mah, GOC:rl Regulation: regulated by regulation of hematopoietic stem cell proliferation [GO:1902033]; negatively regulated by negative regulation of hematopoietic stem cell proliferation [GO:1902034]; positively regulated by positive regulation of hematopoietic stem cell proliferation [GO:1902035]